{
  "gene_name": "Annexin A5",
  "gene": "UniProtKB:P08758",
  "gene_symbol": "ANXA5",
  "term_id": "UNKNOWN:0002",
  "term_label": "Unknown biological process"
}